{
  "term_id": "GO:0005682",
  "term_label": "U5 snRNP",
  "gene_name": "Small nuclear ribonucleoprotein E",
  "gene_symbol": "SNRPE",
  "gene": "UniProtKB:P62304"
}